{
  "gene_symbol": "SHISA9",
  "term_id": "GO:0032281",
  "gene_name": "Protein shisa-9",
  "term_label": "AMPA glutamate receptor complex",
  "gene": "UniProtKB:B4DS77"
}